{
  "gene_symbol": "RFX8",
  "gene": "UniProtKB:Q6ZV50",
  "term_id": "GO:0006357",
  "gene_name": "DNA-binding protein RFX8",
  "term_label": "regulation of transcription by RNA polymerase II"
}